{
  "term_id": "UNKNOWN:0001",
  "gene": "UniProtKB:O60303",
  "gene_name": "Katanin-interacting protein",
  "term_label": "Unknown molecular function",
  "gene_symbol": "KATNIP"
}